regulation of skeletal muscle contraction by neural stimulation via neuromuscular junction [GO:0014852] (BP) Relationships: is a type of regulation of skeletal muscle contraction [GO:0014819] Sources: GOC:ef, GOC:mtg_muscle Definition: Any process that modulates the frequency, rate or extent of skeletal muscle contraction by variation of the pattern of stimulation by nervous system.